{
  "gene_symbol": "PRMT9",
  "term_label": "protein-arginine N-methyltransferase activity",
  "term_id": "GO:0016274",
  "gene_name": "Protein arginine N-methyltransferase 9",
  "gene": "UniProtKB:Q6P2P2"
}